xylose binding [GO:0033222] (molecular function) Sources: GOC:mah Relationships: is_a monosaccharide binding [GO:0048029] Definition: Binding to the D- or L-enantiomer of xylose.